{
  "term_label": "Unknown molecular function",
  "gene": "UniProtKB:Q8NFZ5",
  "gene_symbol": "TNIP2",
  "gene_name": "TNFAIP3-interacting protein 2",
  "term_id": "UNKNOWN:0001"
}